{
  "gene": "UniProtKB:P98164",
  "term_label": "receptor-mediated endocytosis",
  "term_id": "GO:0006898",
  "gene_name": "Low-density lipoprotein receptor-related protein 2",
  "gene_symbol": "LRP2"
}